D-xylulose 5-phosphate metabolic process [GO:0051167] (biological process) Subtypes: GO:0019488, D-arabitol catabolic process to D-xylulose 5-phosphate [GO:0019528], GO:0019569, D-arabinose catabolic process to D-xylulose 5-phosphate [GO:0019573], L-arabitol catabolic process to D-xylulose 5-phosphate [GO:0019590], D-glucuronate catabolic process to D-xylulose 5-phosphate [GO:0019640], formaldehyde assimilation via xylulose monophosphate cycle [GO:0019648], xylitol catabolic process to D-xylulose 5-phosphate [GO:0019697], D-xylulose 5-phosphate biosynthetic process [GO:1901159] Sources: ISBN:0721662544 Also known as: D-xylulose 5-phosphate metabolism, D-xylulose-5-phosphate metabolic process, D-xylulose-5-phosphate metabolism, xylulose 5-phosphate metabolic process, xylulose 5-phosphate metabolism, xylulose-5-phosphate metabolic process, xylulose-5-phosphate metabolism Relationships: is_a phosphate-containing compound metabolic process [GO:0006796]; is_a GO:0019637; is a type of carbohydrate derivative metabolic process [GO:1901135] Definition: The chemical reactions and pathways involving D-xylulose 5-phosphate, a derivative of the ketopentose xylulose phosphorylated at the 5 carbon; it is an intermediate in the pentose phosphate pathway.